positive regulation of response to cell cycle checkpoint signaling [GO:1902146] (biological process) Definition: Any process that activates or increases the frequency, rate or extent of response to cell cycle checkpoint signaling. Sources: GOC:TermGenie, GOC:mtg_cell_cycle Also known as: activation of cell cycle checkpoint effector process, activation of response to signal involved in cell cycle checkpoint, positive regulation of cell cycle checkpoint effector process, positive regulation of response to signal involved in cell cycle checkpoint, up regulation of cell cycle checkpoint effector process, up regulation of response to cell cycle checkpoint signaling, up regulation of response to signal involved in cell cycle checkpoint, up-regulation of cell cycle checkpoint effector process, up-regulation of response to cell cycle checkpoint signaling, up-regulation of response to signal involved in cell cycle checkpoint, upregulation of cell cycle checkpoint effector process, upregulation of response to cell cycle checkpoint signaling, upregulation of response to signal involved in cell cycle checkpoint, activation of response to cell cycle checkpoint signaling, activation of G1/S transition checkpoint effector process, activation of G2/M transition checkpoint effector process, activation of response to G1/S transition checkpoint signaling, activation of response to G2/M transition checkpoint signaling, activation of response to signal involved in G1/S transition checkpoint, activation of response to signal involved in G2/M transition checkpoint, positive regulation of G1/S transition checkpoint effector process, positive regulation of G2/M transition checkpoint effector process, positive regulation of response to G1/S transition checkpoint signaling, positive regulation of response to G2/M transition checkpoint signaling, positive regulation of response to signal involved in G1/S transition checkpoint, positive regulation of response to signal involved in G2/M transition checkpoint, up regulation of G1/S transition checkpoint effector process, up regulation of G2/M transition checkpoint effector process, up regulation of response to G1/S transition checkpoint signaling, up regulation of response to G2/M transition checkpoint signaling, up regulation of response to signal involved in G1/S transition checkpoint, up regulation of response to signal involved in G2/M transition checkpoint, up-regulation of G1/S transition checkpoint effector process, up-regulation of G2/M transition checkpoint effector process, up-regulation of response to G1/S transition checkpoint signaling, up-regulation of response to G2/M transition checkpoint signaling, up-regulation of response to signal involved in G1/S transition checkpoint, up-regulation of response to signal involved in G2/M transition checkpoint, upregulation of G1/S transition checkpoint effector process, upregulation of G2/M transition checkpoint effector process, upregulation of response to G1/S transition checkpoint signaling, upregulation of response to G2/M transition checkpoint signaling, upregulation of response to signal involved in G1/S transition checkpoint, upregulation of response to signal involved in G2/M transition checkpoint Relationships: is_a positive regulation of response to biotic stimulus [GO:0002833]; is a type of positive regulation of cellular process [GO:0048522]; is a type of GO:1902145; positively regulates GO:0072396 Subtypes: positive regulation of response to cytokinesis checkpoint signaling [GO:1902148], positive regulation of response to DNA integrity checkpoint signaling [GO:1902152]